dibenzofuran metabolic process [GO:0018893] (biological process) Also known as: dibenzofuran metabolism Subtypes: dibenzofuran catabolic process [GO:0019340] Definition: The chemical reactions and pathways involving dibenzofuran, a substance composed of two benzene rings linked by one ether bond and one carbon-carbon bond. Dibenzofuran is a white crystalline solid created from the production of coal tar and used as an insecticide and an intermediate in the production of other chemicals. Relationships: is_a small molecule metabolic process [GO:0044281] Sources: GOC:ai, UM-BBD_pathwayID:dbf